{
  "term_label": "synaptic membrane",
  "term_id": "GO:0097060",
  "gene": "UniProtKB:O00408",
  "gene_symbol": "PDE2A",
  "gene_name": "cGMP-dependent 3',5'-cyclic phosphodiesterase"
}